{
  "gene_symbol": "PLA2G4F",
  "term_id": "GO:0046475",
  "gene": "UniProtKB:Q68DD2",
  "gene_name": "Cytosolic phospholipase A2 zeta",
  "term_label": "glycerophospholipid catabolic process"
}